phosphatidylinositol-4-phosphate phosphatase activity [GO:0043812] (molecular function) Also known as: phosphatidylinositol 4-phosphate phosphatase activity Definition: Catalysis of the reaction: a 1,2-diacyl-sn-glycero-3-phospho-(1D-myo-inositol 4-phosphate) + H2O = a 1,2-diacyl-sn-glycero-3-phospho-(1D-myo-inositol) + phosphate. Relationships: is a type of phosphatidylinositol phosphate 4-phosphatase activity [GO:0034596]; is a type of phosphatidylinositol monophosphate phosphatase activity [GO:0052744] References: PMID:10224048 Sources: RHEA:55652